{
  "term_id": "GO:0044027",
  "gene_name": "E3 ubiquitin-protein ligase UHRF1",
  "gene_symbol": "UHRF1",
  "gene": "UniProtKB:Q96T88",
  "term_label": "negative regulation of gene expression via chromosomal CpG island methylation"
}